N-terminal protein amino acid propionylation [GO:0061606] (biological process) References: PMID:17267393, PMID:23043182 Sources: GOC:dph Relationships: is a type of GO:0043687 Definition: The propionylation of the N-terminal amino acid of proteins.